gracilis tract morphogenesis [GO:0021958] (biological process) References: PMID:12867698 Sources: GOC:cls, GOC:dgh, GOC:dph, GOC:jid, GO_REF:0000021 Also known as: tract of Goll morphogenesis Definition: Generation of a long process of a CNS neuron, that carries efferent (outgoing) action potentials from the cell body in the dorsal root ganglion towards target cells in the medulla. This axonal process is a member of those that make up the gracilis tract, a group of axons that are from neurons involved in proprioception from the lower trunk and lower limb. Relationships: is a type of central nervous system projection neuron axonogenesis [GO:0021952]